{
  "gene_symbol": "HMGB1",
  "term_label": "chromatin remodeling",
  "term_id": "GO:0006338",
  "gene": "UniProtKB:P09429",
  "gene_name": "High mobility group protein B1"
}